{
  "gene": "UniProtKB:Q7Z7B7",
  "gene_name": "Beta-defensin 132",
  "term_id": "UNKNOWN:0002",
  "gene_symbol": "DEFB132",
  "term_label": "Unknown biological process"
}